{
  "gene_name": "Protocadherin gamma-A5",
  "gene": "UniProtKB:Q9Y5G8",
  "gene_symbol": "PCDHGA5",
  "term_label": "cell adhesion",
  "term_id": "GO:0007155"
}